{
  "gene": "UniProtKB:P08861",
  "gene_name": "Chymotrypsin-like elastase family member 3B",
  "term_label": "serine-type endopeptidase activity",
  "gene_symbol": "CELA3B",
  "term_id": "GO:0004252"
}